{
  "term_id": "UNKNOWN:0001",
  "gene_name": "Nck-associated protein 5",
  "gene": "UniProtKB:O14513",
  "term_label": "Unknown molecular function",
  "gene_symbol": "NCKAP5"
}